allyl-alcohol dehydrogenase activity [GO:0047655] (molecular function) Definition: Catalysis of the reaction: allyl alcohol + NADP+ = acrolein + H+ + NADPH. Sources: EC:1.1.1.54, RHEA:12168 Also known as: allyl-alcohol:NADP+ oxidoreductase activity Relationships: is a type of GO:0016616